{
  "term_label": "Unknown molecular function",
  "gene": "UniProtKB:O95931",
  "gene_symbol": "CBX7",
  "gene_name": "Chromobox protein homolog 7",
  "term_id": "UNKNOWN:0001"
}